{
  "gene": "UniProtKB:O60513",
  "term_label": "galactosyltransferase activity",
  "term_id": "GO:0008378",
  "gene_name": "Beta-1,4-galactosyltransferase 4",
  "gene_symbol": "B4GALT4"
}